{
  "gene": "UniProtKB:Q5SRR4",
  "term_id": "GO:0009897",
  "term_label": "external side of plasma membrane",
  "gene_symbol": "LY6G5C",
  "gene_name": "Lymphocyte antigen 6 complex locus protein G5c"
}